{
  "term_label": "Unknown biological process",
  "gene_symbol": "MRLN",
  "term_id": "UNKNOWN:0002",
  "gene": "UniProtKB:P0DMT0",
  "gene_name": "Myoregulin"
}